{
  "gene_symbol": "SLX4",
  "gene_name": "Structure-specific endonuclease subunit SLX4",
  "gene": "UniProtKB:Q8IY92",
  "term_id": "UNKNOWN:0001",
  "term_label": "Unknown molecular function"
}